regulation of endoplasmic reticulum stress-induced intrinsic apoptotic signaling pathway [GO:1902235] (biological process) Subtypes: negative regulation of endoplasmic reticulum stress-induced intrinsic apoptotic signaling pathway [GO:1902236], positive regulation of endoplasmic reticulum stress-induced intrinsic apoptotic signaling pathway [GO:1902237], regulation of endoplasmic reticulum stress-induced neuron intrinsic apoptotic signaling pathway [GO:1903381] Relationships: is_a GO:1905897; is a type of regulation of intrinsic apoptotic signaling pathway [GO:2001242]; regulates intrinsic apoptotic signaling pathway in response to endoplasmic reticulum stress [GO:0070059] Also known as: regulation of apoptosis in response to endoplasmic reticulum stress, regulation of ER stress-induced apoptosis, regulation of apoptosis in response to ER stress, regulation of apoptosis triggered by ER stress, regulation of endoplasmic reticulum stress-induced apoptosis, regulation of intrinsic apoptotic signaling pathway in response to endoplasmic reticulum stress, regulation of intrinsic apoptotic signaling pathway induced by endoplasmic reticulum stress References: PMID:20160352 Sources: GOC:BHF, GOC:TermGenie, GOC:mtg_apoptosis, GOC:rl Definition: Any process that modulates the frequency, rate or extent of an endoplasmic reticulum stress-induced intrinsic apoptotic signaling pathway.